{
  "gene": "UniProtKB:Q92673",
  "gene_symbol": "SORL1",
  "term_label": "membrane",
  "term_id": "GO:0016020",
  "gene_name": "Sortilin-related receptor"
}